{
  "gene_name": "Zinc finger and BTB domain-containing protein 39",
  "gene_symbol": "ZBTB39",
  "term_id": "GO:0000122",
  "term_label": "negative regulation of transcription by RNA polymerase II",
  "gene": "UniProtKB:O15060"
}